{
  "term_label": "smoothened signaling pathway",
  "gene": "UniProtKB:P10070",
  "term_id": "GO:0007224",
  "gene_name": "Zinc finger protein GLI2",
  "gene_symbol": "GLI2"
}